lipid binding [GO:0008289] (molecular function) Sources: GOC:ai Definition: Binding to a lipid. Relationships: is a type of binding [GO:0005488] Subtypes: lipopolysaccharide binding [GO:0001530], steroid binding [GO:0005496], fatty acid binding [GO:0005504], phospholipid binding [GO:0005543], triglyceride binding [GO:0017129], isoprenoid binding [GO:0019840], diacylglycerol binding [GO:0019992], GO:0030882, sphingolipid binding [GO:0046625], GO:0051861, GO:0071723, fatty acid derivative binding [GO:1901567] Regulation: negatively regulated by negative regulation of lipid binding [GO:1900131]